positive regulation of opioid receptor signaling pathway [GO:2000476] (biological process) Relationships: is a type of positive regulation of G protein-coupled receptor signaling pathway [GO:0045745]; is a type of regulation of opioid receptor signaling pathway [GO:2000474]; positively regulates G protein-coupled opioid receptor signaling pathway [GO:0038003] Definition: Any process that activates or increases the frequency, rate or extent of opioid receptor signaling pathway. Also known as: positive regulation of opioid receptor signalling pathway Sources: GOC:obol Subtypes: positive regulation of adenylate cyclase-inhibiting opioid receptor signaling pathway [GO:1900731]